galactoside 6-L-fucosyltransferase activity [GO:0046702] (molecular function) Relationships: is a type of alpha-(1->6)-fucosyltransferase activity [GO:0046921] References: PMID:12413479 Definition: Catalysis of the transfer of an L-fucosyl group from GDP-beta-L-fucose to a galactoside acceptor molecule, usually an N-glycan, to form an alpha(1,6)-fucosylated galactoside.